N-acetyllactosaminide beta-1,6-N-acetylglucosaminyltransferase activity [GO:0008109] (molecular function) Definition: Catalysis of the reaction: a beta-D-galactosyl-1,4-N-acetyl-beta-D-glucosaminyl derivative + UDP-N-acetyl-alpha-D-glucosamine = an N-acetyl-beta-D-glucosaminyl-1,6-beta-D-galactosyl-1,4-N-acetyl-beta-D-glucosaminyl derivative + UDP + H+. Sources: RHEA:17413 Also known as: uridine diphosphoacetylglucosamine-acetyllactosaminide beta1->6-acetylglucosaminyltransferase, N-acetylglucosaminyltransferase activity, N-acetyllactosaminide beta-1,6-N-acetylglucosaminyl-transferase activity, UDP-GlcNAc:Gal-R, beta-D-6-N-acetylglucosaminyltransferase activity, UDP-N-acetyl-D-glucosamine:beta-D-galactosyl-1,4-N-acetyl-D-glucosaminide beta-1,6-N-acetyl-D-glucosaminyltransferase activity, galbeta1->4GlcNAc-R beta1->6 N-acetylglucosaminyltransferase activity Relationships: is a type of acetylglucosaminyltransferase activity [GO:0008375]